biotin-CoA ligase activity [GO:0047707] (molecular function) Relationships: is a type of GO:0016405; is a type of GO:0016878 Sources: EC:6.2.1.11, MetaCyc:BIOTIN--COA-LIGASE-RXN Also known as: biotin CoA synthetase activity, biotin:CoA ligase (AMP-forming), biotinyl coenzyme A synthetase activity, biotinyl-CoA synthetase activity Definition: Catalysis of the reaction: ATP + biotin + CoA = AMP + diphosphate + biotinyl-CoA.